{
  "gene": "UniProtKB:P04733",
  "gene_name": "Metallothionein-1F",
  "term_label": "detoxification of copper ion",
  "gene_symbol": "MT1F",
  "term_id": "GO:0010273"
}